{
  "term_label": "Unknown molecular function",
  "gene_name": "GPI transamidase component PIG-S",
  "gene_symbol": "PIGS",
  "term_id": "UNKNOWN:0001",
  "gene": "UniProtKB:Q96S52"
}